{
  "term_label": "Unknown biological process",
  "gene_symbol": "ACTR3B",
  "term_id": "UNKNOWN:0002",
  "gene_name": "Actin-related protein 3B",
  "gene": "UniProtKB:Q9P1U1"
}